{
  "gene": "UniProtKB:P02749",
  "term_label": "Unknown biological process",
  "term_id": "UNKNOWN:0002",
  "gene_name": "Beta-2-glycoprotein 1",
  "gene_symbol": "APOH"
}